{
  "gene_name": "Beta-defensin 135",
  "term_label": "killing of cells of another organism",
  "gene_symbol": "DEFB135",
  "gene": "UniProtKB:Q30KP9",
  "term_id": "GO:0031640"
}